{
  "term_id": "GO:0006895",
  "term_label": "Golgi to endosome transport",
  "gene_name": "Ras-related protein Rab-14",
  "gene_symbol": "RAB14",
  "gene": "UniProtKB:P61106"
}